aminophosphonate metabolic process [GO:0033051] (biological process) Definition: The chemical reactions and pathways involving aminophosphonates, phosphonic acid derivatives that contain an amino group. Also known as: aminophosphonate metabolism Sources: GOC:mah Relationships: is a type of GO:0019637